{
  "gene_symbol": "CDT1",
  "gene_name": "DNA replication factor Cdt1",
  "term_label": "nucleus",
  "term_id": "GO:0005634",
  "gene": "UniProtKB:Q9H211"
}